endothelial tube formation [GO:0120331] (biological process) Relationships: is a type of epithelial tube formation [GO:0072175]; is part of endothelial tube morphogenesis [GO:0061154] Definition: The developmental process pertaining to the initial formation of an endothelial tube. References: PMID:23239824 Sources: GOC:sl